root hair tip [GO:0035619] (cellular component) Definition: The tip portion of an outgrowth of a root epidermal cell. Also known as: root hair cell tip References: PMID:16567499 Relationships: is a type of cell tip [GO:0051286]; is part of root hair [GO:0035618]